{
  "gene_symbol": "XCR1",
  "term_label": "cell chemotaxis",
  "gene_name": "Chemokine XC receptor 1",
  "term_id": "GO:0060326",
  "gene": "UniProtKB:P46094"
}